microtubule lateral binding [GO:0099609] (molecular function) Definition: Binding to the side of a microtubule. Relationships: is a type of microtubule binding [GO:0008017] Sources: GOC:dos